negative regulation of ammonia assimilation cycle [GO:2001249] (BP) Definition: Any process that stops, prevents or reduces the frequency, rate or extent of ammonia assimilation cycle. Also known as: negative regulation of glutamate metabolic process via glutamine and ammonia, negative regulation of glutamate metabolism via glutamine and ammonia Sources: GOC:BHF Relationships: is a type of negative regulation of nitrogen utilization [GO:0045847]; is a type of GO:2000212; is a type of GO:2001248; negatively regulates ammonia assimilation cycle [GO:0019676]